{
  "gene_symbol": "PLGLA",
  "term_label": "Unknown molecular function",
  "gene": "UniProtKB:Q15195",
  "term_id": "UNKNOWN:0001",
  "gene_name": "Plasminogen-like protein A"
}